cardiac muscle cell development [GO:0055013] (biological process) Subtypes: atrial cardiac muscle cell development [GO:0055014], GO:0055015, cardiac pacemaker cell development [GO:0060926] Definition: The process whose specific outcome is the progression of a cardiac muscle cell over time, from its formation to the mature state. Relationships: is a type of GO:0055002; is a type of GO:0055006; is part of GO:0055007 Also known as: cardiac muscle fiber development, cardiac muscle fibre development, cardiomyocyte cell development, heart muscle cell development, heart muscle fiber development Regulation: regulated by regulation of cardiac muscle fiber development [GO:0055018]; negatively regulated by negative regulation of cardiac muscle fiber development [GO:0055019]; positively regulated by positive regulation of cardiac muscle fiber development [GO:0055020] Sources: GOC:devbiol, GOC:mtg_heart